{
  "gene": "UniProtKB:P19367",
  "gene_symbol": "HK1",
  "term_label": "glucose metabolic process",
  "term_id": "GO:0006006",
  "gene_name": "Hexokinase-1"
}